negative regulation of relaxation of cardiac muscle [GO:1901898] (biological process) Relationships: is a type of negative regulation of relaxation of muscle [GO:1901078]; is_a regulation of relaxation of cardiac muscle [GO:1901897]; negatively regulates relaxation of cardiac muscle [GO:0055119] References: PMID:19708671 Sources: GOC:BHF, GOC:TermGenie, GOC:rl Definition: Any process that stops, prevents or reduces the frequency, rate or extent of relaxation of cardiac muscle. Also known as: down regulation of relaxation of cardiac muscle, down-regulation of relaxation of cardiac muscle, downregulation of relaxation of cardiac muscle, inhibition of relaxation of cardiac muscle